{
  "term_label": "mitochondrion organization",
  "gene": "UniProtKB:Q8WYQ3",
  "gene_symbol": "CHCHD10",
  "gene_name": "Coiled-coil-helix-coiled-coil-helix domain-containing protein 10, mitochondrial",
  "term_id": "GO:0007005"
}